{
  "term_id": "GO:0016891",
  "gene": "UniProtKB:Q8N2A8",
  "term_label": "RNA endonuclease activity producing 5'-phosphomonoesters, hydrolytic mechanism",
  "gene_symbol": "PLD6",
  "gene_name": "Mitochondrial cardiolipin hydrolase"
}